{
  "gene_symbol": "CC2D1A",
  "gene": "UniProtKB:Q6P1N0",
  "term_label": "DNA-binding transcription factor activity, RNA polymerase II-specific",
  "gene_name": "Coiled-coil and C2 domain-containing protein 1A",
  "term_id": "GO:0000981"
}